{
  "gene_name": "Potassium voltage-gated channel subfamily D member 1",
  "term_id": "GO:0043025",
  "term_label": "neuronal cell body",
  "gene": "UniProtKB:Q9NSA2",
  "gene_symbol": "KCND1"
}